positive regulation of response to formic acid [GO:1901462] (biological process) Sources: GOC:TermGenie, GOC:mengo_curators Relationships: is a type of positive regulation of response to stimulus [GO:0048584]; is a type of regulation of response to formic acid [GO:1901460]; positively regulates response to formic acid [GO:1901425] Definition: Any process that activates or increases the frequency, rate or extent of response to formic acid. Also known as: up regulation of response to formic acid, up-regulation of response to formic acid, upregulation of response to formic acid, activation of response to formic acid